pseudohyphal septin ring [GO:0032170] (cellular component) Relationships: is a type of GO:0005940 Definition: A tight ring-shaped structure that forms in the division plane at the junction between the mother cell and a pseudohyphal projection; composed of septins as well as septin-associated proteins. References: PMID:16151244 Sources: GOC:krc, GOC:mah